{
  "term_label": "dendrite self-avoidance",
  "term_id": "GO:0070593",
  "gene_symbol": "DSCAM",
  "gene_name": "Cell adhesion molecule DSCAM",
  "gene": "UniProtKB:O60469"
}